rhoptry membrane [GO:0033016] (cellular component) Definition: The lipid bilayer surrounding a rhoptry. Relationships: is a type of organelle membrane [GO:0031090]; is part of GO:0020008 Sources: GOC:mah